{
  "gene": "UniProtKB:Q8N5Z0",
  "term_id": "UNKNOWN:0003",
  "term_label": "Unknown cellular component",
  "gene_symbol": "AADAT",
  "gene_name": "Kynurenine_alpha-aminoadipate aminotransferase, mitochondrial"
}